{
  "term_id": "GO:0030139",
  "gene_symbol": "AMN",
  "gene": "UniProtKB:Q9BXJ7",
  "term_label": "endocytic vesicle",
  "gene_name": "Protein amnionless"
}